mitochondrion autophagosome adaptor activity [GO:0140580] (molecular function) Definition: The binding activity of a molecule that brings together a mitochondrial membrane and an autophagosome during mitophagy. References: PMID:33138913 Relationships: is a type of autophagosome-membrane adaptor activity [GO:0160183] Also known as: mitophagy receptor